{
  "gene": "UniProtKB:O95931",
  "term_id": "GO:0031519",
  "term_label": "PcG protein complex",
  "gene_name": "Chromobox protein homolog 7",
  "gene_symbol": "CBX7"
}